saponin metabolic process [GO:0016134] (biological process) Subtypes: saponin biosynthetic process [GO:0016135], saponin catabolic process [GO:0016136] Definition: The chemical reactions and pathways involving saponins, glycosides of plants in which the aglycan (sapogenin) group is a terpene or steroid and the sugar group is a glucose, a galactose, a pentose, a methylpentose or an oligosaccharide. Saponins are powerful surfactant agents and membrane active; they are, hence, toxic to animals on injection. Relationships: is a type of glycoside metabolic process [GO:0016137] Sources: ISBN:0198547684 Also known as: saponin metabolism